{
  "gene_name": "Trafficking protein particle complex subunit 6A",
  "term_id": "GO:0030008",
  "gene_symbol": "TRAPPC6A",
  "gene": "UniProtKB:O75865",
  "term_label": "TRAPP complex"
}